{
  "gene_symbol": "Q6ZVH6",
  "term_label": "Unknown biological process",
  "gene": "UniProtKB:Q6ZVH6",
  "gene_name": "Putative uncharacterized protein FLJ42569",
  "term_id": "UNKNOWN:0002"
}